{
  "gene_name": "Arf-GAP with coiled-coil, ANK repeat and PH domain-containing protein 3",
  "term_label": "Unknown cellular component",
  "gene": "UniProtKB:Q96P50",
  "term_id": "UNKNOWN:0003",
  "gene_symbol": "ACAP3"
}